zinc efflux transmembrane transporter activity [GO:0022883] (MF) Sources: GOC:mtg_transport, ISBN:0815340729 Relationships: is a type of GO:0005385; is a type of monoatomic cation efflux transmembrane transporter activity [GO:0046583] Also known as: zinc efflux permease activity Definition: Enables the transfer of a zinc ion or zinc ions from the inside of the cell to the outside of the cell across a membrane.